{
  "term_id": "GO:0005222",
  "gene_name": "Cyclic nucleotide-gated cation channel alpha-4",
  "term_label": "intracellularly cAMP-activated cation channel activity",
  "gene_symbol": "CNGA4",
  "gene": "UniProtKB:Q8IV77"
}